alcohol-forming very long-chain fatty acyl-CoA reductase activity [GO:0080019] (molecular function) Also known as: fatty acyl CoA reductase (alcohol-forming) activity, fatty acyl-CoA reductase (alcohol-forming) activity, fatty-acyl-CoA reductase (alcohol-forming) activity Note: While there is not universal consensus on the lengths of short-, medium-, long- and very-long-chain fatty acids, the GO uses the definitions in ChEBI (see CHEBI:26666, CHEBI:59554, CHEBI:15904 and CHEBI:27283). References: PMID:16980563 Sources: RHEA:81751 Relationships: is a type of oxidoreductase activity, acting on the aldehyde or oxo group of donors, NAD or NADP as acceptor [GO:0016620] Definition: Catalysis of the reaction: a very long-chain fatty acyl-CoA + 2 NADPH + 2 H+ = a very long-chain primary fatty alcohol + 2 NADP+ + CoA.